{
  "gene": "UniProtKB:Q9BQE9",
  "term_id": "UNKNOWN:0003",
  "gene_symbol": "BCL7B",
  "gene_name": "B-cell CLL_lymphoma 7 protein family member B",
  "term_label": "Unknown cellular component"
}